acyl-CoA hydrolase activity [GO:0016289] (molecular function) Sources: RHEA:70423 Relationships: is_a thiolester hydrolase activity [GO:0016790]; is a type of deacylase activity [GO:0160215] Definition: Catalysis of the reaction: an acyl-CoA + H2O = a carboxylate + CoA + H+. Subtypes: acetyl-CoA hydrolase activity [GO:0003986], GO:0004778, 4-hydroxybenzoyl-CoA thioesterase activity [GO:0018739], phenylacetyl-CoA hydrolase activity [GO:0033880], choloyl-CoA hydrolase activity [GO:0033882], (S)-methylmalonyl-CoA hydrolase activity [GO:0047511], acetoacetyl-CoA hydrolase activity [GO:0047603], fatty acyl-CoA hydrolase activity [GO:0047617], hydroxymethylglutaryl-CoA hydrolase activity [GO:0047994], GO:0061522 Also known as: CoA hydrolase activity